{
  "gene_symbol": "SHISAL2A",
  "gene_name": "Protein shisa-like-2A",
  "term_label": "Unknown molecular function",
  "gene": "UniProtKB:Q6UWV7",
  "term_id": "UNKNOWN:0001"
}